{
  "gene_name": "Interleukin-1 receptor-like 2",
  "gene_symbol": "IL1RL2",
  "term_label": "cell surface",
  "term_id": "GO:0009986",
  "gene": "UniProtKB:Q9HB29"
}